inhibition of serotonin uptake [GO:0051614] (BP) Relationships: is a type of inhibition of neurotransmitter uptake [GO:0051609]; is a type of negative regulation of serotonin uptake [GO:0051612] Sources: GOC:ai Also known as: inhibition of 5-HT uptake, inhibition of 5-hydroxytryptamine uptake, inhibition of 5HT uptake, inhibition of serotonin import Definition: Any process that prevents the activation of the directed movement of serotonin into a cell.